viral release via pore formation in host cell membrane [GO:0044660] (BP) Also known as: viral exit by cytolysis via pore formation in host cell membrane, viral release by cytolysis via pore formation in host cell membrane, cytolysis by virus via pore formation in host cell membrane Sources: GOC:jl Relationships: is a type of viral release from host cell by cytolysis [GO:0044659]; has part GO:0044658; has part disruption of plasma membrane integrity in another organism [GO:0051673] Definition: The dissemination of mature viral particles from a host cell via the formation by the virus of pores in its host cell membrane.